left lung development [GO:0060459] (BP) Sources: GOC:dph, GOC:mtg_lung Definition: The biological process whose specific outcome is the progression of a left lung from an initial condition to its mature state. This process begins with the formation of the left lung and ends with the mature structure. The left lung is the lung which is on the left side of the anterior posterior axis looking from a dorsal to ventral aspect. Also known as: left pulmonary development Relationships: is a type of lung development [GO:0030324]